{
  "term_id": "GO:0005634",
  "gene_name": "Zinc finger protein 595",
  "term_label": "nucleus",
  "gene_symbol": "ZNF595",
  "gene": "UniProtKB:Q8IYB9"
}